{
  "gene": "UniProtKB:Q9NVR2",
  "term_label": "Unknown molecular function",
  "gene_symbol": "INTS10",
  "term_id": "UNKNOWN:0001",
  "gene_name": "Integrator complex subunit 10"
}